regulation of mRNA cis splicing, via spliceosome [GO:1905744] (biological process) Relationships: is a type of GO:0048024; RO_0002211 mRNA cis splicing, via spliceosome [GO:0045292] References: PMID:2880558 Sources: GOC:TermGenie, GO_REF:0000058 Also known as: regulation of splicing, regulation of nuclear mRNA cis splicing, via spliceosome, regulation of nuclear mRNA cis splicing, via U2-type spliceosome Definition: Any process that modulates the frequency, rate or extent of mRNA cis splicing, via spliceosome. Subtypes: negative regulation of mRNA cis splicing, via spliceosome [GO:1905745], GO:1905746